{
  "term_id": "GO:0070915",
  "gene": "UniProtKB:Q92633",
  "term_label": "lysophosphatidic acid receptor activity",
  "gene_name": "Lysophosphatidic acid receptor 1",
  "gene_symbol": "LPAR1"
}